{
  "gene": "UniProtKB:P46939",
  "term_label": "plasma membrane",
  "gene_symbol": "UTRN",
  "gene_name": "Utrophin",
  "term_id": "GO:0005886"
}